2-oxoglutaramate amidase activity [GO:0106008] (molecular function) References: PMID:21288482 Sources: EC:3.5.1.111 Definition: Catalysis of the reaction: 2-oxoglutaramate + H2O = 2-oxoglutarate + NH3. Relationships: is a type of GO:0016811